{
  "gene_symbol": "EPC1",
  "term_label": "chromatin organization",
  "gene": "UniProtKB:Q9H2F5",
  "term_id": "GO:0006325",
  "gene_name": "Enhancer of polycomb homolog 1"
}